polynucleotide 3' dephosphorylation [GO:0098506] (BP) Relationships: is a type of nucleobase-containing compound metabolic process [GO:0006139]; is a type of GO:0016311; is a type of macromolecule metabolic process [GO:0043170] Definition: The process of removing one or more phosphate groups from the 3' end of a polynucleotide. Sources: GOC:dos